{
  "gene_name": "G-protein coupled receptor 52",
  "gene_symbol": "GPR52",
  "gene": "UniProtKB:Q9Y2T5",
  "term_label": "phototransduction",
  "term_id": "GO:0007602"
}